{
  "gene_name": "Coiled-coil domain-containing protein 194",
  "term_id": "UNKNOWN:0001",
  "gene": "UniProtKB:A0A1B0GVG4",
  "gene_symbol": "CCDC194",
  "term_label": "Unknown molecular function"
}